regulation of cell motility [GO:2000145] (biological process) Definition: Any process that modulates the frequency, rate or extent of cell motility. Also known as: regulation of cell locomotion, regulation of movement of a cell, regulation of cell movement Subtypes: regulation of cell migration [GO:0030334], regulation of cilium-dependent cell motility [GO:1902019], GO:1902021, GO:1905416, negative regulation of cell motility [GO:2000146], positive regulation of cell motility [GO:2000147] Relationships: is a type of regulation of locomotion [GO:0040012]; is a type of GO:0050794; regulates cell motility [GO:0048870] Sources: GOC:mah